Cvt vesicle membrane [GO:0033110] (cellular component) Relationships: is_a GO:0030659; is part of Cvt vesicle [GO:0033107] References: PMID:20065092 Sources: GOC:ecd Definition: Either of the two lipid bilayers surrounding a Cvt vesicle, a vesicle that functions in the cytoplasm-to-vacuole targeting (Cvt) pathway. Also known as: cytoplasm to vacuole targeting vesicle membrane, cytoplasm-to-vacuole targeting vesicle membrane